{
  "term_label": "G1/S transition of mitotic cell cycle",
  "term_id": "GO:0000082",
  "gene_symbol": "GPR132",
  "gene": "UniProtKB:Q9UNW8",
  "gene_name": "Probable G-protein coupled receptor 132"
}